{
  "term_label": "centrosome",
  "gene_name": "Serine_threonine-protein kinase Nek2",
  "gene": "UniProtKB:P51955",
  "term_id": "GO:0005813",
  "gene_symbol": "NEK2"
}